{
  "term_label": "L-proline import across plasma membrane",
  "gene_symbol": "SLC6A20",
  "gene": "UniProtKB:Q9NP91",
  "gene_name": "Sodium- and chloride-dependent transporter XTRP3",
  "term_id": "GO:1904271"
}